{
  "gene_name": "Cytochrome b-c1 complex subunit 2, mitochondrial",
  "term_label": "respiratory chain complex III",
  "term_id": "GO:0045275",
  "gene": "UniProtKB:P22695",
  "gene_symbol": "UQCRC2"
}